{
  "gene_symbol": "MMS22L",
  "gene": "UniProtKB:Q6ZRQ5",
  "term_id": "UNKNOWN:0001",
  "gene_name": "Protein MMS22-like",
  "term_label": "Unknown molecular function"
}